{
  "term_label": "regulation of actin filament polymerization",
  "term_id": "GO:0030833",
  "gene_name": "Rho GTPase-activating protein 40",
  "gene": "UniProtKB:Q5TG30",
  "gene_symbol": "ARHGAP40"
}